{
  "gene_name": "DNA transposase THAP9",
  "gene": "UniProtKB:Q9H5L6",
  "term_id": "GO:0004803",
  "gene_symbol": "THAP9",
  "term_label": "transposase activity"
}